{
  "term_label": "proteoglycan biosynthetic process",
  "term_id": "GO:0030166",
  "gene": "UniProtKB:Q9UBV7",
  "gene_name": "Beta-1,4-galactosyltransferase 7",
  "gene_symbol": "B4GALT7"
}